{
  "gene_name": "Solute carrier family 12 member 6",
  "term_label": "cell volume homeostasis",
  "term_id": "GO:0006884",
  "gene": "UniProtKB:Q9UHW9",
  "gene_symbol": "SLC12A6"
}